acetoin dehydrogenase (NAD+) activity [GO:0019152] (molecular function) Definition: Catalysis of the reaction: acetoin + NAD+ = diacetyl + NADH + H+. This reaction is catalyzed in the reverse direction. Also known as: diacetyl reductase activity Subtypes: diacetyl reductase ((R)-acetoin forming) (NAD+) activity [GO:0052587], diacetyl reductase ((S)-acetoin forming) (NAD+) activity [GO:0052588] Sources: MetaCyc:ACETOINDEHYDROG-RXN Relationships: is a type of GO:0016616